{
  "term_id": "GO:0005634",
  "gene_name": "E3 ubiquitin-protein transferase RMND5B",
  "gene": "UniProtKB:Q96G75",
  "term_label": "nucleus",
  "gene_symbol": "RMND5B"
}